{
  "gene": "UniProtKB:P14209",
  "gene_name": "CD99 antigen",
  "gene_symbol": "CD99",
  "term_id": "GO:0005886",
  "term_label": "plasma membrane"
}